{
  "gene": "UniProtKB:P41208",
  "term_id": "GO:0006289",
  "term_label": "nucleotide-excision repair",
  "gene_name": "Centrin-2",
  "gene_symbol": "CETN2"
}